{
  "term_id": "GO:0097038",
  "gene_name": "Oxysterol-binding protein-related protein 3",
  "gene": "UniProtKB:Q9H4L5",
  "gene_symbol": "OSBPL3",
  "term_label": "perinuclear endoplasmic reticulum"
}